positive regulation of biomineral tissue development [GO:0070169] (biological process) Sources: GOC:mah Subtypes: positive regulation of bone mineralization [GO:0030501], positive regulation of tooth mineralization [GO:0070172], positive regulation of shell calcification [GO:1905650] Relationships: is a type of positive regulation of developmental process [GO:0051094]; is a type of GO:0070167; positively regulates GO:0031214 Definition: Any process that activates or increases the frequency, rate or extent of biomineral tissue development, the formation of hard tissues that consist mainly of inorganic compounds.